copper chelate transmembrane transporter activity [GO:0051981] (molecular function) Subtypes: copper-nicotianamine transmembrane transporter activity [GO:0051982] Definition: Enables the transfer of a copper chelate from one side of a membrane to the other. A copper chelate is a heterocyclic compound having a metal ion attached by coordinate bonds to at least two nonmetal ions. References: PMID:26512647 Relationships: is a type of copper ion transmembrane transporter activity [GO:0005375]